{
  "gene": "UniProtKB:P02686",
  "term_label": "neuronal cell body",
  "term_id": "GO:0043025",
  "gene_symbol": "MBP",
  "gene_name": "Myelin basic protein"
}